{
  "gene_symbol": "SULT6B1",
  "term_id": "GO:0051923",
  "term_label": "sulfation",
  "gene_name": "Sulfotransferase 6B1",
  "gene": "UniProtKB:Q6IMI4"
}